{
  "gene": "UniProtKB:F8WBI6",
  "gene_name": "Golgin subfamily A member 8N",
  "gene_symbol": "GOLGA8N",
  "term_label": "Golgi cis cisterna",
  "term_id": "GO:0000137"
}